polysaccharide metabolic process [GO:0005976] (biological process) Also known as: polysaccharide metabolism, glycan metabolic process, glycan metabolism, multicellular organismal polysaccharide metabolic process Regulation: regulated by GO:0032881 Subtypes: GO:0000271, polysaccharide catabolic process [GO:0000272], substituted mannan metabolic process [GO:0006080], GO:0010383, galacturonan metabolic process [GO:0010393], arabinan metabolic process [GO:0031221], GO:0044042, xylan metabolic process [GO:0045491], GO:0046378, alginic acid acetylation [GO:0051979] Sources: ISBN:0198547684 Relationships: is a type of carbohydrate metabolic process [GO:0005975]; is a type of macromolecule metabolic process [GO:0043170] Definition: The chemical reactions and pathways involving a polysaccharide, a polymer of many (typically more than 10) monosaccharide residues linked glycosidically.